3-chlorocatechol catabolic process [GO:1901168] (biological process) Relationships: is a type of catechol-containing compound catabolic process [GO:0019614]; is a type of benzene-containing compound metabolic process [GO:0042537]; is a type of GO:0090345 Definition: The chemical reactions and pathways resulting in the breakdown of 3-chlorocatechol. Also known as: 3-chlorocatechol breakdown, 3-chlorocatechol catabolism, 3-chlorocatechol degradation Sources: GOC:TermGenie, GOC:yaf, UniPathway:UPA00083